synaptic vesicle exocytosis [GO:0016079] (biological process) Sources: GOC:jid, GOC:lmg Definition: Fusion of intracellular membrane-bounded vesicles with the pre-synaptic membrane of the neuronal cell resulting in release of neurotransmitter into the synaptic cleft. Regulation: regulated by GO:2000300; negatively regulated by GO:2000301; positively regulated by positive regulation of synaptic vesicle exocytosis [GO:2000302] Relationships: is a type of regulated exocytosis [GO:0045055]; is_a GO:0051649; is a type of vesicle-mediated transport in synapse [GO:0099003]; is a type of signal release from synapse [GO:0099643]; is part of neurotransmitter secretion [GO:0007269]; is part of synaptic vesicle cycle [GO:0099504]; occurs in presynapse [GO:0098793] Subtypes: calcium ion-regulated exocytosis of neurotransmitter [GO:0048791], spontaneous exocytosis of neurotransmitter [GO:0048792]